{
  "gene_name": "ENTH domain-containing protein 1",
  "gene": "UniProtKB:Q8IYW4",
  "term_label": "phospholipid binding",
  "term_id": "GO:0005543",
  "gene_symbol": "ENTHD1"
}